{
  "gene": "UniProtKB:Q9UK17",
  "term_label": "action potential",
  "gene_name": "Potassium voltage-gated channel subfamily D member 3",
  "gene_symbol": "KCND3",
  "term_id": "GO:0001508"
}